{
  "gene_symbol": "LY86",
  "term_id": "GO:0045087",
  "gene_name": "Lymphocyte antigen 86",
  "gene": "UniProtKB:O95711",
  "term_label": "innate immune response"
}